pyrimidine nucleoside transport [GO:0015864] (biological process) Subtypes: GO:0015861, uridine transmembrane transport [GO:0015862] Regulation: regulated by regulation of pyrimidine nucleoside transport [GO:0032246] Definition: The directed movement of a pyrimidine nucleoside, a pyrimidine base covalently bonded to a ribose or deoxyribose sugar, into, out of or within a cell, or between cells, by means of some agent such as a transporter or pore. Relationships: is a type of nucleoside transport [GO:0015858] Sources: GOC:ai